nuclear-transcribed mRNA catabolic process, deadenylation-dependent decay [GO:0000288] (biological process) Definition: A major pathway of degradation of nuclear-transcribed mRNAs that proceeds through a series of ordered steps that includes poly(A) tail shortening and that can regulate mRNA stability. Sources: GOC:jp, GOC:krc Also known as: deadenylation-dependent mRNA decay, mRNA breakdown, deadenylation-dependent decay, mRNA catabolic process, deadenylation-dependent, mRNA catabolic process, deadenylylation-dependent, mRNA catabolism, deadenylation-dependent, mRNA catabolism, deadenylylation-dependent, mRNA degradation, deadenylation-dependent decay, nuclear mRNA catabolic process, deadenylation-dependent decay Relationships: is a type of nuclear-transcribed mRNA catabolic process [GO:0000956]; is a type of mRNA destabilization [GO:0061157] Regulation: regulated by regulation of nuclear-transcribed mRNA catabolic process, deadenylation-dependent decay [GO:1900151]; negatively regulated by negative regulation of nuclear-transcribed mRNA catabolic process, deadenylation-dependent decay [GO:1900152]; RO_0002213 by positive regulation of nuclear-transcribed mRNA catabolic process, deadenylation-dependent decay [GO:1900153]